{
  "gene_name": "Transmembrane protein 229A",
  "gene_symbol": "TMEM229A",
  "gene": "UniProtKB:B2RXF0",
  "term_label": "Unknown molecular function",
  "term_id": "UNKNOWN:0001"
}